{
  "term_label": "Unknown molecular function",
  "term_id": "UNKNOWN:0001",
  "gene": "UniProtKB:P26436",
  "gene_symbol": "ACRV1",
  "gene_name": "Acrosomal protein SP-10"
}